glucosylglycerol 3-phosphatase activity [GO:0050530] (molecular function) Sources: EC:3.1.3.69, RHEA:22652 Also known as: 2-(beta-D-glucosyl)-sn-glycerol-3-phosphate phosphohydrolase activity, StpA, salt tolerance protein A Definition: Catalysis of the reaction: 2-O-(beta-D-glucosyl)-sn-glycerol 3-phosphate + H2O = 2-O-(beta-D-glucosyl)-sn-glycerol + phosphate. Relationships: is a type of phosphatase activity [GO:0016791]